{
  "gene_name": "Homeobox protein MSX-1",
  "term_label": "RNA polymerase II transcription regulatory region sequence-specific DNA binding",
  "term_id": "GO:0000977",
  "gene": "UniProtKB:P28360",
  "gene_symbol": "MSX1"
}